{
  "term_id": "GO:0003729",
  "gene_symbol": "CIRBP",
  "gene_name": "Cold-inducible RNA-binding protein",
  "term_label": "mRNA binding",
  "gene": "UniProtKB:Q14011"
}